{
  "gene_name": "IF rod domain-containing protein",
  "term_label": "intermediate filament organization",
  "gene": "UniProtKB:A0A140TA62",
  "gene_symbol": "LOC100653049",
  "term_id": "GO:0045109"
}